post-embryonic genitalia morphogenesis [GO:0035126] (biological process) Subtypes: imaginal disc-derived genitalia morphogenesis [GO:0048805] Definition: The process, occurring after embryonic development, by which the anatomical structures of the genitalia are generated and organized. Also known as: post-embryonic genital morphogenesis Sources: GOC:bf Relationships: is a type of GO:0035112